{
  "gene_symbol": "ATP8A1",
  "gene": "UniProtKB:Q9Y2Q0",
  "term_label": "phospholipid translocation",
  "term_id": "GO:0045332",
  "gene_name": "Phospholipid-transporting ATPase IA"
}